{
  "gene": "UniProtKB:O43639",
  "term_id": "GO:0035591",
  "term_label": "signaling adaptor activity",
  "gene_symbol": "NCK2",
  "gene_name": "Cytoplasmic protein NCK2"
}